limb spinous cell differentiation [GO:0060890] (biological process) Sources: GOC:dph, GOC:sdb_2009, GOC:tb Definition: The process in which a relatively unspecialized cell acquires specialized features of a limb epidermal spinous cell. Relationships: is a type of keratinocyte differentiation [GO:0030216]; is part of limb epidermis development [GO:0060887]